{
  "term_id": "UNKNOWN:0002",
  "gene_name": "GH3 domain-containing protein",
  "term_label": "Unknown biological process",
  "gene": "UniProtKB:Q8N2G8",
  "gene_symbol": "GHDC"
}